{
  "gene_symbol": "RCOR3",
  "gene_name": "REST corepressor 3",
  "gene": "UniProtKB:Q9P2K3",
  "term_id": "GO:0000118",
  "term_label": "histone deacetylase complex"
}